{
  "gene": "UniProtKB:P10144",
  "gene_symbol": "GZMB",
  "gene_name": "Granzyme B",
  "term_label": "protein maturation",
  "term_id": "GO:0051604"
}